{
  "term_label": "olfactory receptor activity",
  "gene": "UniProtKB:Q96R72",
  "gene_name": "Olfactory receptor 4K3",
  "gene_symbol": "OR4K3",
  "term_id": "GO:0004984"
}